{
  "term_id": "GO:0000977",
  "gene_symbol": "HAND2",
  "gene_name": "Heart- and neural crest derivatives-expressed protein 2",
  "gene": "UniProtKB:P61296",
  "term_label": "RNA polymerase II transcription regulatory region sequence-specific DNA binding"
}